{
  "term_id": "UNKNOWN:0002",
  "gene_symbol": "PAQR6",
  "term_label": "Unknown biological process",
  "gene": "UniProtKB:Q6TCH4",
  "gene_name": "Membrane progestin receptor delta"
}